nucleic acid binding [GO:0003676] (molecular function) Relationships: is a type of binding [GO:0005488] Subtypes: transcription regulatory region nucleic acid binding [GO:0001067], DNA binding [GO:0003677], RNA binding [GO:0003723], DNA/RNA hybrid binding [GO:0071667], annealing activity [GO:0140666] Definition: Binding to a nucleic acid. Also known as: base pairing Sources: GOC:jl